{
  "term_label": "Unknown cellular component",
  "gene": "UniProtKB:Q96H35",
  "gene_symbol": "RBM18",
  "gene_name": "Probable RNA-binding protein 18",
  "term_id": "UNKNOWN:0003"
}